protein trans-autophosphorylation [GO:0036290] (biological process) Also known as: trans-autophosphorylation Subtypes: GO:1990579 Definition: The phosphorylation by a protein of a residue on an identical protein. For example, phosphorylation by the other kinase within a homodimer. Relationships: is a type of protein autophosphorylation [GO:0046777] References: PMID:20516151 Sources: GOC:jsg